{
  "term_label": "negative regulation of DNA-templated transcription",
  "term_id": "GO:0045892",
  "gene": "UniProtKB:Q9NP08",
  "gene_symbol": "HMX1",
  "gene_name": "Homeobox protein HMX1"
}